{
  "gene_name": "Myosin-10",
  "term_id": "GO:0032982",
  "gene_symbol": "MYH10",
  "gene": "UniProtKB:P35580",
  "term_label": "myosin filament"
}